Pip2-Oaf1 complex [GO:0089716] (cellular component) References: PMID:8972187, PMID:9288897 Relationships: is a type of RNA polymerase II transcription regulator complex [GO:0090575] Definition: A heterodimeric complex consisting of Zn(2)Cys(6) containing transcription factors Pip2 and Oaf1. It binds to the oleate response element (ORE), found in the promoters of fatty acid-inducible genes in Saccharomyces where, in the presence of oleate this bound complex activates the transcription of genes encoding peroxisomal proteins.